regulation of chloroplast fission [GO:1905192] (biological process) Definition: Any process that modulates the frequency, rate or extent of chloroplast fission. References: PMID:26862170 Sources: GOC:TermGenie, GO_REF:0000058 Also known as: regulation of chloroplast division Note: Any process that modulates the rate, frequency or extent of chloroplast fission. Chloroplast fission is the division of a chloroplast within a cell to form two or more separate chloroplast compartments. Relationships: is a type of regulation of organelle organization [GO:0033043]; regulates chloroplast fission [GO:0010020] Subtypes: GO:1905193, positive regulation of chloroplast fission [GO:1905194]